negative regulation of sporangiospore formation [GO:0075288] (biological process) Definition: Any process that stops, prevents, or reduces the frequency, rate or extent of sporangiospore formation, a process in which sporangiospores, a type of asexual spore found in fungi, are formed. Sporangiospores are formed within sac-like structure, the sporangium, following the division of the cytoplasm. Sources: GOC:pamgo_curators Subtypes: negative regulation of zoospore formation [GO:0075242], GO:0075292 Relationships: is a type of negative regulation of asexual sporulation resulting in formation of a cellular spore [GO:0043944]; is a type of regulation of sporangiospore formation [GO:0075286]; negatively regulates sporangiospore formation [GO:0034300]